{
  "gene": "UniProtKB:Q96PQ7",
  "term_id": "GO:0031463",
  "gene_symbol": "KLHL5",
  "term_label": "Cul3-RING ubiquitin ligase complex",
  "gene_name": "Kelch-like protein 5"
}